{
  "gene_name": "Thioredoxin reductase 2, mitochondrial",
  "gene": "UniProtKB:Q9NNW7",
  "gene_symbol": "TXNRD2",
  "term_label": "cell redox homeostasis",
  "term_id": "GO:0045454"
}